{
  "gene_symbol": "NUDT15",
  "gene": "UniProtKB:Q9NV35",
  "term_label": "cytosol",
  "term_id": "GO:0005829",
  "gene_name": "Nucleotide triphosphate diphosphatase NUDT15"
}